{
  "term_id": "GO:0032396",
  "gene_symbol": "LILRA1",
  "gene": "UniProtKB:O75019",
  "gene_name": "Leukocyte immunoglobulin-like receptor subfamily A member 1",
  "term_label": "inhibitory MHC class I receptor activity"
}